{
  "term_id": "GO:0015026",
  "gene_name": "Receptor activity-modifying protein 2",
  "term_label": "coreceptor activity",
  "gene_symbol": "RAMP2",
  "gene": "UniProtKB:O60895"
}